{
  "gene_symbol": "TM4SF1",
  "gene_name": "Transmembrane 4 L6 family member 1",
  "term_id": "GO:0016020",
  "term_label": "membrane",
  "gene": "UniProtKB:P30408"
}